{
  "gene_name": "GPALPP motifs-containing protein 1",
  "term_label": "Unknown cellular component",
  "gene_symbol": "GPALPP1",
  "gene": "UniProtKB:Q8IXQ4",
  "term_id": "UNKNOWN:0003"
}